DNA damage response, signal transduction by p53 class mediator [GO:0030330] (biological process) Definition: A cascade of processes induced by the cell cycle regulator phosphoprotein p53, or an equivalent protein, in response to the detection of DNA damage. Sources: GOC:go_curators Also known as: p53-mediated DNA damage response, DNA damage response, activation of p53, TP53 signaling pathway, p53 signaling pathway Relationships: is a type of signal transduction in response to DNA damage [GO:0042770]; is a type of signal transduction by p53 class mediator [GO:0072331] Regulation: regulated by GO:0043516; positively regulated by GO:0043517; negatively regulated by GO:0043518